{
  "gene_symbol": "NDFIP2",
  "term_id": "GO:0031398",
  "gene_name": "NEDD4 family-interacting protein 2",
  "gene": "UniProtKB:Q9NV92",
  "term_label": "positive regulation of protein ubiquitination"
}